{
  "gene_symbol": "C3orf36",
  "term_id": "UNKNOWN:0001",
  "term_label": "Unknown molecular function",
  "gene_name": "Uncharacterized protein C3orf36",
  "gene": "UniProtKB:Q3SXR2"
}